{
  "gene_symbol": "MARCHF11",
  "gene_name": "E3 ubiquitin-protein ligase MARCHF11",
  "term_id": "UNKNOWN:0003",
  "gene": "UniProtKB:A6NNE9",
  "term_label": "Unknown cellular component"
}